{
  "term_id": "GO:0000978",
  "gene_name": "Lymphoid enhancer-binding factor 1",
  "gene": "UniProtKB:Q9UJU2",
  "term_label": "RNA polymerase II cis-regulatory region sequence-specific DNA binding",
  "gene_symbol": "LEF1"
}